hydroxylysine kinase activity [GO:0047992] (MF) Also known as: GTP:5-hydroxy-L-lysine O-phosphotransferase activity, guanosine triphosphate:5-hydroxy-L-lysine O-phosphotransferase activity, hydroxylysine kinase (phosphorylating) Sources: EC:2.7.1.81, RHEA:19049 Relationships: is a type of phosphotransferase activity, alcohol group as acceptor [GO:0016773]; is a type of amino acid kinase activity [GO:0019202] Definition: Catalysis of the reaction: erythro-5-hydroxy-L-lysine + GTP = 5-phosphonooxy-L-lysine + GDP + 2 H+.